{
  "gene_name": "Early placenta insulin-like peptide",
  "gene_symbol": "INSL4",
  "term_label": "Unknown biological process",
  "gene": "UniProtKB:Q14641",
  "term_id": "UNKNOWN:0002"
}